caffeate O-methyltransferase activity [GO:0047763] (molecular function) Sources: EC:2.1.1.68 Definition: Catalysis of the reaction: S-adenosyl-L-methionine + 3,4-dihydroxy-trans-cinnamate = S-adenosyl-L-homocysteine + 3-methoxy-4-hydroxy-trans-cinnamate. Also known as: S-adenosyl-L-methionine:3,4-dihydroxy-trans-cinnamate 3-O-methyltransferase activity, S-adenosyl-L-methionine:caffeic acid-O-methyltransferase activity, caffeate 3-O-methyltransferase activity, caffeate methyltransferase activity Relationships: is a type of O-methyltransferase activity [GO:0008171]